{
  "gene_symbol": "SERPINA11",
  "term_label": "extracellular space",
  "gene": "UniProtKB:Q86U17",
  "term_id": "GO:0005615",
  "gene_name": "Serpin A11"
}